polyol biosynthetic process [GO:0046173] (biological process) Definition: The chemical reactions and pathways resulting in the formation of a polyol, any alcohol containing three or more hydroxyl groups attached to saturated carbon atoms. Relationships: is a type of polyol metabolic process [GO:0019751]; is a type of alcohol biosynthetic process [GO:0046165] Subtypes: inositol biosynthetic process [GO:0006021], GO:0019401, streptomycin biosynthetic process [GO:0019872], inositol phosphate biosynthetic process [GO:0032958], diol biosynthetic process [GO:0034312], GO:0036378, phytosphingosine biosynthetic process [GO:0071602], phenolic phthiocerol biosynthetic process [GO:0097041], vomitoxin biosynthetic process [GO:0106110], resolvin biosynthetic process [GO:0106295], GO:0140880, GO:1901121, gentamycin biosynthetic process [GO:1901130], kanamycin biosynthetic process [GO:1901133], vistamycin biosynthetic process [GO:1901152], GO:1901155, neomycin biosynthetic process [GO:1901158], GO:1901744, butirosin biosynthetic process [GO:1901758], 1,5-anhydro-D-fructose biosynthetic process [GO:1901803] Also known as: polyhydric alcohol biosynthetic process, polyol anabolism, polyol biosynthesis, polyol formation, polyol synthesis Sources: GOC:curators